{
  "gene": "UniProtKB:Q14571",
  "term_label": "calcium ion binding",
  "term_id": "GO:0005509",
  "gene_symbol": "ITPR2",
  "gene_name": "Inositol 1,4,5-trisphosphate receptor type 2"
}